{
  "gene": "UniProtKB:Q9HCE7",
  "term_label": "ubiquitin protein ligase activity",
  "gene_symbol": "SMURF1",
  "term_id": "GO:0061630",
  "gene_name": "E3 ubiquitin-protein ligase SMURF1"
}